{
  "term_label": "plasma membrane",
  "gene_symbol": "PIK3CA",
  "gene_name": "Phosphatidylinositol 4,5-bisphosphate 3-kinase catalytic subunit alpha isoform",
  "gene": "UniProtKB:P42336",
  "term_id": "GO:0005886"
}